{
  "term_id": "GO:0008374",
  "gene": "UniProtKB:Q8NCC3",
  "term_label": "O-acyltransferase activity",
  "gene_symbol": "PLA2G15",
  "gene_name": "Phospholipase A2 group XV"
}